UTP-C complex [GO:0034456] (cellular component) Note: Note that the term name uses Saccharomyces gene product names because no other names have yet arisen for this complex; the term nevertheless can be used for analogous complexes in other eukaryotes, and the name can be changed if better wording is found. Also known as: Rrp7p-containing subcomplex of 90S preribosome Relationships: is a type of nuclear protein-containing complex [GO:0140513]; is part of nucleolus [GO:0005730]; is part of GO:0030686 References: PMID:17515605 Sources: GOC:mah Definition: A protein complex that forms a subcomplex of the 90S preribosome. In S. cerevisiae, it is composed of Rrp7p, Utp22p, Ckb1p, Cka1p, Ckb2p and Cka2p.